{
  "gene": "UniProtKB:Q15761",
  "term_id": "GO:0005886",
  "gene_symbol": "NPY5R",
  "term_label": "plasma membrane",
  "gene_name": "Neuropeptide Y receptor type 5"
}